response to glutathione [GO:1901370] (biological process) Sources: GOC:TermGenie Definition: Any process that results in a change in state or activity of a cell or an organism (in terms of movement, secretion, enzyme production, gene expression, etc.) as a result of a glutathione stimulus. Subtypes: cellular response to glutathione [GO:0072753] Relationships: is_a response to nitrogen compound [GO:1901698]; is a type of response to oxygen-containing compound [GO:1901700]